{
  "gene_symbol": "AGTR2",
  "gene_name": "Type-2 angiotensin II receptor",
  "gene": "UniProtKB:P50052",
  "term_label": "inflammatory response",
  "term_id": "GO:0006954"
}